{
  "gene_name": "Transcription factor BTF3",
  "gene": "UniProtKB:P20290",
  "term_id": "GO:0005829",
  "term_label": "cytosol",
  "gene_symbol": "BTF3"
}